tartrate transmembrane transport [GO:0015745] (biological process) Also known as: tartrate transport Relationships: is a type of transmembrane transport [GO:0055085] Definition: The process in which tartrate is transported across a lipid bilayer, from one side of a membrane to the other. Sources: GOC:krc